{
  "gene": "UniProtKB:Q9BZS1",
  "term_label": "RNA polymerase II cis-regulatory region sequence-specific DNA binding",
  "gene_name": "Forkhead box protein P3",
  "term_id": "GO:0000978",
  "gene_symbol": "FOXP3"
}